monoatomic anion transmembrane transporter activity [GO:0008509] (molecular function) Relationships: is_a GO:0015075; BFO_0000050 monoatomic anion transmembrane transport [GO:0098656] Also known as: anion transmembrane transporter activity, anion transporter activity Definition: Enables the transfer of a negatively charged ion from one side of a membrane to the other. Subtypes: monoatomic anion channel activity [GO:0005253], folate:monoatomic anion antiporter activity [GO:0008518], GO:0015108, GO:0015111, GO:0015296, orotate:monoatomic anion antiporter activity [GO:0140812], urate:monoatomic anion antiporter activity [GO:0140813], bicarbonate:monoatomic anion antiporter activity [GO:0140829], GO:1903425 Sources: GOC:dgf, GOC:mtg_transport, ISBN:0815340729